cAMP transport [GO:0070730] (BP) Sources: GOC:mah, ISBN:0198506732 Also known as: cyclic AMP transport Relationships: is a type of organic anion transport [GO:0015711]; is a type of purine ribonucleotide transport [GO:0015868]; is a type of adenine nucleotide transport [GO:0051503]; is a type of cyclic nucleotide transport [GO:0070729] Definition: The directed movement of cyclic AMP (cAMP), into, out of or within a cell.